{
  "gene": "UniProtKB:P17035",
  "term_label": "DNA-binding transcription factor activity, RNA polymerase II-specific",
  "gene_symbol": "ZNF28",
  "term_id": "GO:0000981",
  "gene_name": "Zinc finger protein 28"
}